{
  "gene_name": "Putative uncharacterized protein encoded by BRWD1-AS2",
  "term_label": "Unknown biological process",
  "gene": "UniProtKB:P59051",
  "gene_symbol": "BRWD1-AS2",
  "term_id": "UNKNOWN:0002"
}